allulose 6-phosphate 3-epimerase activity [GO:0034700] (molecular function) Definition: Catalysis of the reaction: D-allulose 6-phosphate = keto-D-fructose 6-phosphate. Relationships: is a type of GO:0016857 Sources: RHEA:28426